{
  "gene_symbol": "KRT17",
  "term_label": "cytoskeleton",
  "gene_name": "Keratin, type I cytoskeletal 17",
  "term_id": "GO:0005856",
  "gene": "UniProtKB:Q04695"
}